{
  "term_label": "postsynapse",
  "gene_name": "Gamma-aminobutyric acid receptor subunit alpha-1",
  "gene": "UniProtKB:P14867",
  "term_id": "GO:0098794",
  "gene_symbol": "GABRA1"
}